{
  "term_id": "GO:0000398",
  "gene_name": "U6 snRNA-associated Sm-like protein LSm3",
  "gene_symbol": "LSM3",
  "gene": "UniProtKB:P62310",
  "term_label": "mRNA splicing, via spliceosome"
}